immature T cell proliferation [GO:0033079] (biological process) Sources: GOC:add, ISBN:0781735149 Subtypes: GO:0033080 Regulation: regulated by GO:0033083; negatively regulated by negative regulation of immature T cell proliferation [GO:0033087]; positively regulated by positive regulation of immature T cell proliferation [GO:0033091] Relationships: is a type of T cell proliferation [GO:0042098] Definition: The expansion of an immature T cell population by cell division.